water transport [GO:0006833] (biological process) Definition: The directed movement of water (H2O) into, out of or within a cell, or between cells, by means of some agent such as a transporter or pore. Relationships: is a type of fluid transport [GO:0042044] Sources: GOC:ai Subtypes: renal water transport [GO:0003097], pollen hydration [GO:0009859], transpiration [GO:0010148], transepithelial water transport [GO:0035377]